{
  "term_id": "GO:0003677",
  "gene_name": "Major centromere autoantigen B",
  "gene": "UniProtKB:P07199",
  "gene_symbol": "CENPB",
  "term_label": "DNA binding"
}